{
  "term_id": "GO:0050431",
  "gene_symbol": "WFIKKN2",
  "term_label": "transforming growth factor beta binding",
  "gene": "UniProtKB:Q8TEU8",
  "gene_name": "WAP, Kazal, immunoglobulin, Kunitz and NTR domain-containing protein 2"
}